positive regulation of haustorium mother cell formation [GO:0075194] (biological process) Sources: GOC:pamgo_curators Definition: Any process that activates or increases the frequency, rate or extent of symbiont haustorium mother cell formation. The host is defined as the larger of the organisms involved in a symbiotic interaction. Relationships: is a type of GO:0051094; is a type of regulation of haustorium mother cell formation [GO:0075193]; positively regulates haustorium mother cell formation [GO:0075192] Note: Note that this term should not be used to annotate gene products of the host. It should only be used to annotate those gene products from the symbiont involved in this process. Also known as: positive regulation of haustorium mother cell formation on or near host